{
  "term_label": "tight junction assembly",
  "gene_name": "InaD-like protein",
  "gene": "UniProtKB:Q8NI35",
  "term_id": "GO:0120192",
  "gene_symbol": "PATJ"
}